{
  "gene_symbol": "PLEKHF1",
  "term_label": "endosome to lysosome transport",
  "gene_name": "Pleckstrin homology domain-containing family F member 1",
  "term_id": "GO:0008333",
  "gene": "UniProtKB:Q96S99"
}